{
  "gene_name": "AN1-type zinc finger protein 6",
  "term_label": "protein targeting to peroxisome",
  "gene_symbol": "ZFAND6",
  "term_id": "GO:0006625",
  "gene": "UniProtKB:Q6FIF0"
}